{
  "term_id": "UNKNOWN:0001",
  "gene": "UniProtKB:P0DJ93",
  "term_label": "Unknown molecular function",
  "gene_symbol": "SMIM13",
  "gene_name": "Small integral membrane protein 13"
}